{
  "gene_name": "Lactoperoxidase",
  "term_id": "GO:0042742",
  "term_label": "defense response to bacterium",
  "gene_symbol": "LPO",
  "gene": "UniProtKB:P22079"
}